lymphangiogenesis [GO:0001946] (biological process) Relationships: is a type of anatomical structure morphogenesis [GO:0009653]; is a type of anatomical structure formation involved in morphogenesis [GO:0048646]; is part of lymph vessel morphogenesis [GO:0036303] Regulation: regulated by regulation of lymphangiogenesis [GO:1901490]; RO_0002212 by negative regulation of lymphangiogenesis [GO:1901491]; positively regulated by positive regulation of lymphangiogenesis [GO:1901492] Also known as: lymph vessel formation Definition: Lymph vessel formation when new vessels emerge from the proliferation of pre-existing vessels. References: PMID:11596157 Sources: GOC:dph